negative regulation of neural crest cell fate specification [GO:1905296] (biological process) Relationships: is a type of negative regulation of cell fate specification [GO:0009996]; is a type of GO:0090301; is a type of negative regulation of neural crest cell differentiation [GO:1905293]; is_a GO:1905295; negatively regulates neural crest cell fate specification [GO:0014036] Also known as: down regulation of neural crest cell fate specification, down-regulation of neural crest cell fate specification, downregulation of neural crest cell fate specification, inhibition of neural crest cell fate specification Definition: Any process that stops, prevents or reduces the frequency, rate or extent of neural crest cell fate specification. References: PMID:15073157 Sources: GOC:BHF, GOC:TermGenie, GOC:rl, GO_REF:0000058